{
  "term_label": "Golgi apparatus",
  "gene_symbol": "GPR107",
  "term_id": "GO:0005794",
  "gene": "UniProtKB:Q5VW38",
  "gene_name": "Protein GPR107"
}